nucleoside bisphosphate metabolic process [GO:0033865] (biological process) Definition: The chemical reactions and pathways involving a nucleoside bisphosphate, a compound consisting of a nucleobase linked to a deoxyribose or ribose sugar esterified with one phosphate group attached to each of two different hydroxyl groups on the sugar. Relationships: is a type of nucleoside phosphate metabolic process [GO:0006753] Sources: GOC:mah, GOC:pde Subtypes: GO:0033866, nucleoside bisphosphate catabolic process [GO:0033869], ribonucleoside bisphosphate metabolic process [GO:0033875], purine nucleoside bisphosphate metabolic process [GO:0034032] Also known as: nucleoside bisphosphate metabolism